{
  "term_id": "GO:0061630",
  "gene_name": "Baculoviral IAP repeat-containing protein 7",
  "gene_symbol": "BIRC7",
  "term_label": "ubiquitin protein ligase activity",
  "gene": "UniProtKB:Q96CA5"
}